{
  "gene_symbol": "EXOSC8",
  "term_id": "GO:0000176",
  "gene_name": "Exosome complex component RRP43",
  "term_label": "nuclear exosome (RNase complex)",
  "gene": "UniProtKB:Q96B26"
}